nitrate assimilation [GO:0042128] (BP) Definition: The nitrogen metabolic process that encompasses the uptake of nitrate from the environment and reduction to ammonia, and results in the incorporation of nitrogen derived from nitrate into cellular substances. References: PMID:10542156, PMID:8122899 Sources: GOC:das, GOC:mah Also known as: assimilatory nitrate reduction Regulation: regulated by regulation of nitrate assimilation [GO:0090352] Relationships: is_a nitrate metabolic process [GO:0042126]; is a type of nitrogen cycle metabolic process [GO:0071941]; BFO_0000051 nitrate transmembrane transporter activity [GO:0015112]; has part nitrite reductase activity [GO:0098809]